ecdysone binding [GO:0035100] (molecular function) Definition: Binding to 20-hydroxyecdysone (ecdysone). Ecdysone is an ecdysteroid produced by the prothoracic glands of immature insects and the ovaries of adult females, which stimulates growth and molting. Relationships: is a type of GO:0032934; is a type of hormone binding [GO:0042562]; is a type of GO:0043178 Sources: GOC:bf, ISBN:0198506732, ISBN:0582227089